vestibular receptor cell morphogenesis [GO:0060116] (biological process) Definition: Any process that alters the size or shape of a vestibular receptor cell. Sources: GOC:dph, GOC:tb Also known as: vestibular hair cell morphogenesis Relationships: is_a embryonic morphogenesis [GO:0048598]; is a type of GO:0048667; is part of inner ear morphogenesis [GO:0042472]; is part of vestibular receptor cell development [GO:0060118]